{
  "term_label": "cholesterol homeostasis",
  "gene": "UniProtKB:O15118",
  "term_id": "GO:0042632",
  "gene_symbol": "NPC1",
  "gene_name": "NPC intracellular cholesterol transporter 1"
}